{
  "term_label": "Unknown molecular function",
  "gene_symbol": "XAB2",
  "term_id": "UNKNOWN:0001",
  "gene_name": "Pre-mRNA-splicing factor SYF1",
  "gene": "UniProtKB:Q9HCS7"
}